{
  "gene_symbol": "H2BC15",
  "term_label": "chromatin organization",
  "gene": "UniProtKB:Q99877",
  "gene_name": "Histone H2B type 1-N",
  "term_id": "GO:0006325"
}